lysosome organization [GO:0007040] (biological process) Relationships: is a type of lytic vacuole organization [GO:0080171] Also known as: lysosome organisation, lysosome organization and biogenesis Regulation: regulated by regulation of lysosome organization [GO:1905671]; RO_0002212 by negative regulation of lysosome organization [GO:1905672]; positively regulated by GO:1905673 Sources: GOC:mah Definition: A process that is carried out at the cellular level which results in the assembly, arrangement of constituent parts, or disassembly of a lysosome. A lysosome is a cytoplasmic, membrane-bounded organelle that is found in most animal cells and that contains a variety of hydrolases. Subtypes: phagolysosome assembly [GO:0001845]